cellular response to streptomycin [GO:0071239] (biological process) Sources: GOC:mah Definition: Any process that results in a change in state or activity of a cell (in terms of movement, secretion, enzyme production, gene expression, etc.) as a result of a streptomycin stimulus. Streptomycin is a commonly used antibiotic in cell culture media which acts only on prokaryotes and blocks transition from initiation complex to chain elongating ribosome. Relationships: is a type of GO:0046679; is a type of cellular response to antibiotic [GO:0071236]; is a type of cellular response to oxygen-containing compound [GO:1901701]